{
  "term_label": "extracellular space",
  "gene": "UniProtKB:Q8WWU7",
  "gene_symbol": "ITLN2",
  "term_id": "GO:0005615",
  "gene_name": "Intelectin-2"
}